{
  "gene_name": "NADP-dependent malic enzyme, mitochondrial",
  "gene_symbol": "ME3",
  "term_label": "malate dehydrogenase (decarboxylating) (NADP+) activity",
  "term_id": "GO:0004473",
  "gene": "UniProtKB:Q16798"
}